{
  "gene_symbol": "SYPL1",
  "gene_name": "Synaptophysin-like protein 1",
  "gene": "UniProtKB:Q16563",
  "term_label": "Unknown biological process",
  "term_id": "UNKNOWN:0002"
}